{
  "gene_name": "Plexin-A2",
  "term_id": "GO:0071526",
  "term_label": "semaphorin-plexin signaling pathway",
  "gene_symbol": "PLXNA2",
  "gene": "UniProtKB:O75051"
}